axonal fasciculation [GO:0007413] (biological process) Also known as: fasciculation of neuron Relationships: is_a neuron recognition [GO:0008038]; is a type of neuron projection fasciculation [GO:0106030]; is part of axon development [GO:0061564] Subtypes: GO:0097155, GO:0097156 Definition: The collection of axons into a bundle of rods, known as a fascicle. Sources: GOC:dgh